{
  "gene_name": "DNA replication complex GINS protein PSF3",
  "term_label": "Unknown molecular function",
  "term_id": "UNKNOWN:0001",
  "gene_symbol": "GINS3",
  "gene": "UniProtKB:Q9BRX5"
}